{
  "term_id": "GO:0035556",
  "gene_name": "Serine_threonine-protein kinase WNK2",
  "gene_symbol": "WNK2",
  "term_label": "intracellular signal transduction",
  "gene": "UniProtKB:Q9Y3S1"
}